{
  "term_label": "receptor clustering",
  "gene_name": "Membrane-associated guanylate kinase, WW and PDZ domain-containing protein 2",
  "term_id": "GO:0043113",
  "gene_symbol": "MAGI2",
  "gene": "UniProtKB:Q86UL8"
}